{
  "gene_symbol": "U2AF2",
  "term_label": "poly-pyrimidine tract binding",
  "gene": "UniProtKB:P26368",
  "term_id": "GO:0008187",
  "gene_name": "Splicing factor U2AF 65 kDa subunit"
}